cellular response to dinitrophenol [GO:1904642] (biological process) Definition: Any process that results in a change in state or activity of a cell (in terms of movement, secretion, enzyme production, gene expression, etc.) as a result of a dinitrophenol stimulus. References: PMID:24336883 Sources: GOC:TermGenie, GO_REF:0000071 Relationships: is a type of cellular response to nitrogen compound [GO:1901699]; is a type of GO:1901701; is a type of GO:1904641 Also known as: cellular response to dinitrophenols